{
  "gene_name": "Cytotoxic granule associated RNA binding protein TIA1",
  "gene_symbol": "TIA1",
  "term_label": "protein-RNA adaptor activity",
  "gene": "UniProtKB:P31483",
  "term_id": "GO:0140517"
}